{
  "term_id": "UNKNOWN:0001",
  "gene_name": "Centromere protein T",
  "gene": "UniProtKB:Q96BT3",
  "gene_symbol": "CENPT",
  "term_label": "Unknown molecular function"
}